regulation of blood vessel branching [GO:1905553] (biological process) References: PMID:23201774 Sources: GOC:BHF, GOC:BHF_telomere, GOC:TermGenie, GOC:nc, GO_REF:0000058 Also known as: regulation of branching involved in blood vessel morphogenesis Relationships: is a type of GO:0045765; is a type of GO:0060688; is a type of GO:1905330; regulates branching involved in blood vessel morphogenesis [GO:0001569] Subtypes: negative regulation of blood vessel branching [GO:1905554], positive regulation of blood vessel branching [GO:1905555] Definition: Any process that modulates the frequency, rate or extent of blood vessel branching.